{
  "term_label": "Unknown molecular function",
  "gene": "UniProtKB:Q8N9L7",
  "gene_symbol": "Q8N9L7",
  "gene_name": "Putative uncharacterized protein FLJ36925",
  "term_id": "UNKNOWN:0001"
}